{
  "gene": "UniProtKB:Q96AJ9",
  "gene_name": "Vesicle transport through interaction with t-SNAREs homolog 1A",
  "term_label": "SNARE binding",
  "gene_symbol": "VTI1A",
  "term_id": "GO:0000149"
}